{
  "term_label": "plasma membrane",
  "gene_symbol": "PIPSL",
  "gene_name": "Putative PIP5K1A and PSMD4-like protein",
  "gene": "UniProtKB:A2A3N6",
  "term_id": "GO:0005886"
}